peptidyl-lysine desuccinylation [GO:0036049] (biological process) Definition: The removal of a succinyl group (CO-CH2-CH2-CO) from a succinylated lysine residue in a peptide or protein. References: PMID:22076378 Sources: GOC:sp Relationships: is a type of peptidyl-lysine modification [GO:0018205]; is a type of protein desuccinylation [GO:0036048]